{
  "term_id": "UNKNOWN:0002",
  "term_label": "Unknown biological process",
  "gene_name": "Transmembrane 4 L6 family member 19",
  "gene_symbol": "TM4SF19",
  "gene": "UniProtKB:Q96DZ7"
}